{
  "gene": "UniProtKB:P42574",
  "gene_name": "Caspase-3",
  "gene_symbol": "CASP3",
  "term_id": "GO:0043525",
  "term_label": "positive regulation of neuron apoptotic process"
}